{
  "gene": "UniProtKB:Q5VUG0",
  "gene_symbol": "SFMBT2",
  "term_label": "histone binding",
  "term_id": "GO:0042393",
  "gene_name": "Scm-like with four MBT domains protein 2"
}